{
  "gene_name": "Superoxide dismutase [Cu-Zn]",
  "term_id": "GO:0005507",
  "gene": "UniProtKB:P00441",
  "gene_symbol": "SOD1",
  "term_label": "copper ion binding"
}